positive regulation of T cell differentiation [GO:0045582] (biological process) Sources: GOC:go_curators Also known as: positive regulation of T lymphocyte differentiation, positive regulation of T-cell differentiation, positive regulation of T-lymphocyte differentiation, up regulation of T cell differentiation, up-regulation of T cell differentiation, upregulation of T cell differentiation, activation of T cell differentiation, stimulation of T cell differentiation, positive regulation of T cell development Definition: Any process that activates or increases the frequency, rate or extent of T cell differentiation. Subtypes: GO:0033089, positive regulation of extrathymic T cell differentiation [GO:0033090], positive regulation of memory T cell differentiation [GO:0043382], GO:0045585, positive regulation of gamma-delta T cell differentiation [GO:0045588], positive regulation of regulatory T cell differentiation [GO:0045591], positive regulation of alpha-beta T cell differentiation [GO:0046638], positive regulation of pro-T cell differentiation [GO:2000176] Relationships: is a type of regulation of T cell differentiation [GO:0045580]; is a type of positive regulation of lymphocyte differentiation [GO:0045621]; is a type of positive regulation of T cell activation [GO:0050870]; positively regulates T cell differentiation [GO:0030217] Note: Note that immunologists typically use the word 'development' to refer to cells of B or T cell lineages undergoing the process that GO describes as 'cell differentiation'.